{
  "gene_name": "Homer protein homolog 1",
  "term_label": "postsynaptic density",
  "gene_symbol": "HOMER1",
  "term_id": "GO:0014069",
  "gene": "UniProtKB:Q86YM7"
}